T cell secretory granule organization [GO:0033371] (biological process) Definition: A process that is carried out at the cellular level which results in the assembly, arrangement of constituent parts, or disassembly of a secretory granule in a T cell. A secretory granule is a small subcellular vesicle, surrounded by a membrane, that is formed from the Golgi apparatus and contains a highly concentrated protein destined for secretion. Relationships: is a type of secretory granule organization [GO:0033363] Also known as: T cell secretory granule organisation, T lymphocyte secretory granule organization, T-cell secretory granule organization, T-lymphocyte secretory granule organization, T cell secretory granule organization and biogenesis, T-lymphocyte secretory granule maturation Sources: GOC:mah